{
  "term_label": "intermediate filament cytoskeleton organization",
  "gene_name": "Envoplakin",
  "gene_symbol": "EVPL",
  "gene": "UniProtKB:Q92817",
  "term_id": "GO:0045104"
}